{
  "gene": "UniProtKB:Q8NH74",
  "term_id": "GO:0005886",
  "term_label": "plasma membrane",
  "gene_symbol": "OR10A6",
  "gene_name": "Olfactory receptor 10A6"
}